ATP-dependent polynucleotide 5'-hydroxyl-kinase activity [GO:0051734] (molecular function) Sources: EC:2.7.1.78 Subtypes: ATP-dependent polydeoxyribonucleotide 5'-hydroxyl-kinase activity [GO:0046404], ATP-dependent polyribonucleotide 5'-hydroxyl-kinase activity [GO:0051736] Also known as: polynucleotide kinase activity, ATP-dependent polynucleotide kinase activity Relationships: is_a GO:0051731 Definition: Catalysis of the reaction: ATP + 5'-dephosphopolynucleotide = ADP + 5'-phosphopolynucleotide. The polynucleotide may be DNA or RNA.